{
  "gene_name": "Catenin alpha-2",
  "gene": "UniProtKB:P26232",
  "term_label": "beta-catenin binding",
  "gene_symbol": "CTNNA2",
  "term_id": "GO:0008013"
}